{
  "gene_name": "Acyl-CoA dehydrogenase family member 11",
  "term_label": "acyl-CoA dehydrogenase activity",
  "term_id": "GO:0003995",
  "gene_symbol": "ACAD11",
  "gene": "UniProtKB:Q709F0"
}